{
  "gene": "UniProtKB:P46439",
  "term_label": "glutathione transferase activity",
  "gene_symbol": "GSTM5",
  "gene_name": "Glutathione S-transferase Mu 5",
  "term_id": "GO:0004364"
}